{
  "gene": "UniProtKB:Q6QHK4",
  "gene_symbol": "FIGLA",
  "term_label": "Unknown cellular component",
  "term_id": "UNKNOWN:0003",
  "gene_name": "Factor in the germline alpha"
}